{
  "gene_name": "Zinc finger BED domain-containing protein 4",
  "gene": "UniProtKB:O75132",
  "gene_symbol": "ZBED4",
  "term_label": "Unknown molecular function",
  "term_id": "UNKNOWN:0001"
}